{
  "term_label": "nucleus",
  "gene_name": "tRNA (cytosine(38)-C(5))-methyltransferase",
  "term_id": "GO:0005634",
  "gene": "UniProtKB:O14717",
  "gene_symbol": "TRDMT1"
}